{
  "gene_name": "Olfactory receptor 4K3",
  "term_id": "UNKNOWN:0003",
  "term_label": "Unknown cellular component",
  "gene": "UniProtKB:Q96R72",
  "gene_symbol": "OR4K3"
}